{
  "gene_name": "Ras-related protein Rab-6A",
  "term_id": "GO:0006890",
  "gene": "UniProtKB:P20340",
  "term_label": "retrograde vesicle-mediated transport, Golgi to endoplasmic reticulum",
  "gene_symbol": "RAB6A"
}